{
  "term_id": "UNKNOWN:0003",
  "gene_symbol": "TSFM",
  "gene": "UniProtKB:P43897",
  "term_label": "Unknown cellular component",
  "gene_name": "Elongation factor Ts, mitochondrial"
}